{
  "gene": "UniProtKB:O14653",
  "term_id": "GO:0006891",
  "term_label": "intra-Golgi vesicle-mediated transport",
  "gene_name": "Golgi SNAP receptor complex member 2",
  "gene_symbol": "GOSR2"
}